{
  "term_label": "Unknown cellular component",
  "gene_name": "Uncharacterized protein",
  "gene": "UniProtKB:A0A6Q8PGS0",
  "term_id": "UNKNOWN:0003",
  "gene_symbol": "A0A6Q8PGS0"
}